{
  "gene_symbol": "IFNA8",
  "gene_name": "Interferon alpha-8",
  "term_id": "GO:0005125",
  "term_label": "cytokine activity",
  "gene": "UniProtKB:P32881"
}